{
  "gene": "UniProtKB:P19320",
  "gene_symbol": "VCAM1",
  "gene_name": "Vascular cell adhesion protein 1",
  "term_label": "cell adhesion",
  "term_id": "GO:0007155"
}